{
  "term_label": "glial cell-derived neurotrophic factor receptor signaling pathway",
  "term_id": "GO:0035860",
  "gene": "UniProtKB:Q5T4W7",
  "gene_symbol": "ARTN",
  "gene_name": "Artemin"
}